{
  "term_label": "endogenous lipid antigen binding",
  "gene": "UniProtKB:P15812",
  "gene_name": "T-cell surface glycoprotein CD1e, membrane-associated",
  "gene_symbol": "CD1E",
  "term_id": "GO:0030883"
}